{
  "term_id": "GO:0005634",
  "term_label": "nucleus",
  "gene": "UniProtKB:Q09028",
  "gene_symbol": "RBBP4",
  "gene_name": "Histone-binding protein RBBP4"
}